{
  "gene": "UniProtKB:Q6DHV7",
  "term_label": "inosine biosynthetic process",
  "term_id": "GO:0046103",
  "gene_symbol": "MAPDA",
  "gene_name": "Adenosine deaminase-like protein"
}